{
  "gene_name": "Ras-related protein Rab-35",
  "gene": "UniProtKB:Q15286",
  "term_id": "GO:0005525",
  "term_label": "GTP binding",
  "gene_symbol": "RAB35"
}